{
  "term_label": "Unknown biological process",
  "gene": "UniProtKB:Q9H5Z1",
  "gene_symbol": "DHX35",
  "gene_name": "Probable ATP-dependent RNA helicase DHX35",
  "term_id": "UNKNOWN:0002"
}